{
  "gene_symbol": "CUL5",
  "term_id": "GO:0019005",
  "term_label": "SCF ubiquitin ligase complex",
  "gene_name": "Cullin-5",
  "gene": "UniProtKB:Q93034"
}